protoheme IX farnesyltransferase activity [GO:0008495] (molecular function) Sources: RHEA:28070 Also known as: haem O synthase activity, heme A:farnesyltransferase activity, heme O synthase activity, protohaem IX farnesyltransferase activity Definition: Catalysis of the reaction: protoheme IX + (2E,6E)-farnesyl diphosphate + H2O = heme O + diphosphate. Relationships: is a type of GO:0004659